{
  "term_id": "GO:0007043",
  "gene_name": "Cadherin-17",
  "gene": "UniProtKB:Q12864",
  "gene_symbol": "CDH17",
  "term_label": "cell-cell junction assembly"
}